{
  "gene_symbol": "ARSD",
  "term_id": "UNKNOWN:0002",
  "term_label": "Unknown biological process",
  "gene_name": "Arylsulfatase D",
  "gene": "UniProtKB:P51689"
}